inositol phosphoceramide metabolic process [GO:0006673] (BP) Subtypes: mannosyl-inositol phosphorylceramide metabolic process [GO:0006675], mannosyl diphosphorylinositol ceramide metabolic process [GO:0006676] Relationships: is_a GO:0006644; is a type of GO:0006665 Also known as: inositol phosphorylceramide metabolic process, inositol phosphorylceramide metabolism, inositolphosphoceramide metabolism Definition: The chemical reactions and pathways involving inositol phosphoceramides, any lipid with a phosphodiester bridge between an inositol residue and the ceramide group. References: PMID:19726565